{
  "term_id": "GO:0015267",
  "gene_symbol": "AQP12A",
  "term_label": "channel activity",
  "gene": "UniProtKB:Q8IXF9",
  "gene_name": "Aquaporin-12A"
}